positive regulation of protein localization to cell division site involved in mitotic actomyosin contractile ring assembly [GO:0110083] (biological process) Definition: Any process that activates or increases the frequency, rate or extent of protein localization to cell division site involved in mitotic actomyosin contractile ring assembly. Relationships: is a type of regulation of protein localization to cell division site involved in mitotic actomyosin contractile ring assembly [GO:0110082]; is a type of positive regulation of protein localization [GO:1903829]; positively regulates protein localization to cell division site involved in mitotic actomyosin contractile ring assembly [GO:1903476] References: PMID:29343550 Sources: GOC:vw